positive regulation of nucleobase-containing compound transport [GO:0032241] (biological process) Sources: GOC:mah Subtypes: positive regulation of nucleoside transport [GO:0032244], positive regulation of hypoxanthine transport [GO:0035346], positive regulation of thymine transport [GO:0035367], positive regulation of RNA import into nucleus [GO:0046830], positive regulation of RNA export from nucleus [GO:0046833] Also known as: up regulation of nucleobase, nucleoside, nucleotide and nucleic acid transport, up-regulation of nucleobase, nucleoside, nucleotide and nucleic acid transport, upregulation of nucleobase, nucleoside, nucleotide and nucleic acid transport, activation of nucleobase, nucleoside, nucleotide and nucleic acid transport, stimulation of nucleobase, nucleoside, nucleotide and nucleic acid transport, positive regulation of nucleobase, nucleoside, nucleotide and nucleic acid transport Relationships: is a type of regulation of nucleobase-containing compound transport [GO:0032239]; is a type of positive regulation of transport [GO:0051050]; positively regulates nucleobase-containing compound transport [GO:0015931] Definition: Any process that activates or increases the frequency, rate or extent of the directed movement of nucleobases, nucleosides, nucleotides and nucleic acids, into, out of or within a cell, or between cells, by means of some agent such as a transporter or pore.